{
  "term_label": "phosphatidate phosphatase activity",
  "gene": "UniProtKB:Q8TBJ4",
  "gene_name": "Phospholipid phosphatase-related protein type 1",
  "gene_symbol": "PLPPR1",
  "term_id": "GO:0008195"
}